{
  "term_label": "detoxification of copper ion",
  "gene_symbol": "MT4",
  "term_id": "GO:0010273",
  "gene": "UniProtKB:P47944",
  "gene_name": "Metallothionein-4"
}